{
  "gene_name": "Solute carrier family 12 member 2",
  "term_label": "potassium ion import across plasma membrane",
  "gene_symbol": "SLC12A2",
  "gene": "UniProtKB:P55011",
  "term_id": "GO:1990573"
}